{
  "gene_symbol": "URB1-AS1",
  "term_id": "UNKNOWN:0001",
  "gene_name": "Putative uncharacterized protein URB1-AS1",
  "term_label": "Unknown molecular function",
  "gene": "UniProtKB:Q96HZ7"
}